{
  "gene_name": "Membrane-spanning 4-domains subfamily A member 5",
  "gene_symbol": "MS4A5",
  "gene": "UniProtKB:Q9H3V2",
  "term_label": "cell surface receptor signaling pathway",
  "term_id": "GO:0007166"
}